{
  "term_label": "ionotropic glutamate receptor binding",
  "gene_name": "Disks large homolog 1",
  "term_id": "GO:0035255",
  "gene": "UniProtKB:Q12959",
  "gene_symbol": "DLG1"
}